{
  "gene": "UniProtKB:Q8IYI8",
  "term_id": "GO:0000981",
  "gene_symbol": "ZNF440",
  "gene_name": "Zinc finger protein 440",
  "term_label": "DNA-binding transcription factor activity, RNA polymerase II-specific"
}